{
  "term_label": "protein-macromolecule adaptor activity",
  "gene_name": "PDZ domain-containing protein 11",
  "gene_symbol": "PDZD11",
  "term_id": "GO:0030674",
  "gene": "UniProtKB:Q5EBL8"
}